dibenzofuran 4,4a-dioxygenase activity [GO:0018610] (molecular function) Relationships: is a type of GO:0016708 Sources: MetaCyc:R606-RXN, RHEA:42460 Definition: Catalysis of the reaction: dibenzofuran + NADH + H+ + O2 = 2,2',3-trihydroxybiphenyl + NAD+.